{
  "gene_symbol": "BTF3",
  "gene_name": "Transcription factor BTF3",
  "term_id": "UNKNOWN:0001",
  "gene": "UniProtKB:P20290",
  "term_label": "Unknown molecular function"
}